{
  "gene": "UniProtKB:P46094",
  "term_id": "GO:0009897",
  "gene_name": "Chemokine XC receptor 1",
  "gene_symbol": "XCR1",
  "term_label": "external side of plasma membrane"
}